hypolemmal cisterna [GO:1990039] (cellular component) Definition: Specialized part of the smooth endoplasmic reticulum that closely underlies the plasma membrane, usually within 60 nm or closer. Sources: ISBN:0195065719, NIF_Subcellular:sao1634374950 Also known as: hypolemmal cisternae Relationships: is a type of smooth endoplasmic reticulum cisterna [GO:0120082] Subtypes: sub-surface cisterna [GO:1990040]